{
  "gene_name": "Protein shisa-2 homolog",
  "term_label": "endoplasmic reticulum",
  "gene": "UniProtKB:Q6UWI4",
  "gene_symbol": "SHISA2",
  "term_id": "GO:0005783"
}